{
  "gene_symbol": "MYLK",
  "term_id": "GO:0005737",
  "gene_name": "Myosin light chain kinase, smooth muscle",
  "gene": "UniProtKB:Q15746",
  "term_label": "cytoplasm"
}